{
  "gene_symbol": "ZNF563",
  "term_label": "regulation of transcription by RNA polymerase II",
  "gene_name": "Zinc finger protein 563",
  "term_id": "GO:0006357",
  "gene": "UniProtKB:Q8TA94"
}